{
  "gene": "UniProtKB:Q7Z3J2",
  "gene_name": "VPS35 endosomal protein-sorting factor-like",
  "gene_symbol": "VPS35L",
  "term_id": "UNKNOWN:0001",
  "term_label": "Unknown molecular function"
}